{
  "gene_name": "Angiotensin-converting enzyme",
  "term_label": "metallopeptidase activity",
  "gene": "UniProtKB:P12821",
  "term_id": "GO:0008237",
  "gene_symbol": "ACE"
}